{
  "term_id": "UNKNOWN:0002",
  "gene": "UniProtKB:Q9UL45",
  "gene_symbol": "BLOC1S6",
  "gene_name": "Biogenesis of lysosome-related organelles complex 1 subunit 6",
  "term_label": "Unknown biological process"
}